cellular response to interleukin-4 [GO:0071353] (biological process) Sources: GOC:mah Relationships: is a type of GO:0070670; is a type of cellular response to cytokine stimulus [GO:0071345] Definition: Any process that results in a change in state or activity of a cell (in terms of movement, secretion, enzyme production, gene expression, etc.) as a result of an interleukin-4 stimulus. Also known as: cellular response to IL-4